{
  "gene": "UniProtKB:Q13526",
  "term_id": "GO:0005829",
  "gene_name": "Peptidyl-prolyl cis-trans isomerase NIMA-interacting 1",
  "term_label": "cytosol",
  "gene_symbol": "PIN1"
}